{
  "gene_symbol": "GRAMD2A",
  "term_label": "endoplasmic reticulum-plasma membrane tethering",
  "gene": "UniProtKB:Q8IUY3",
  "term_id": "GO:0061817",
  "gene_name": "GRAM domain-containing protein 2A"
}